{
  "gene": "UniProtKB:Q6ZWK4",
  "term_label": "plasma membrane",
  "gene_name": "Regulator of hemoglobinization and erythroid cell expansion protein",
  "term_id": "GO:0005886",
  "gene_symbol": "RHEX"
}